{
  "term_id": "GO:0009952",
  "gene_name": "Transcription factor HES-2",
  "gene_symbol": "HES2",
  "term_label": "anterior/posterior pattern specification",
  "gene": "UniProtKB:Q9Y543"
}